{
  "gene_name": "UDP-N-acetylhexosamine pyrophosphorylase-like protein 1",
  "gene_symbol": "UAP1L1",
  "term_label": "UDP-N-acetylglucosamine biosynthetic process",
  "gene": "UniProtKB:Q3KQV9",
  "term_id": "GO:0006048"
}